{
  "gene_name": "DNA-directed RNA polymerase I subunit RPA43",
  "gene": "UniProtKB:Q3B726",
  "term_id": "GO:0005736",
  "term_label": "RNA polymerase I complex",
  "gene_symbol": "POLR1F"
}